positive regulation of T cell tolerance induction [GO:0002666] (biological process) Sources: GOC:add Relationships: is a type of positive regulation of tolerance induction [GO:0002645]; is a type of regulation of T cell tolerance induction [GO:0002664]; positively regulates T cell tolerance induction [GO:0002517] Also known as: positive regulation of T lymphocyte tolerance induction, positive regulation of T-cell tolerance induction, positive regulation of T-lymphocyte tolerance induction, up regulation of T cell tolerance induction, up-regulation of T cell tolerance induction, upregulation of T cell tolerance induction, activation of T cell tolerance induction, stimulation of T cell tolerance induction Definition: Any process that activates or increases the frequency, rate, or extent of T cell tolerance induction. Subtypes: positive regulation of T cell anergy [GO:0002669], positive regulation of peripheral T cell tolerance induction [GO:0002851]